{
  "term_label": "cytosol",
  "gene": "UniProtKB:Q9UEW8",
  "term_id": "GO:0005829",
  "gene_symbol": "STK39",
  "gene_name": "STE20_SPS1-related proline-alanine-rich protein kinase"
}